{
  "gene": "UniProtKB:O95841",
  "term_label": "extracellular space",
  "gene_name": "Angiopoietin-related protein 1",
  "gene_symbol": "ANGPTL1",
  "term_id": "GO:0005615"
}